{
  "term_label": "negative regulation of small GTPase mediated signal transduction",
  "gene_symbol": "ARHGAP17",
  "term_id": "GO:0051058",
  "gene": "UniProtKB:Q68EM7",
  "gene_name": "Rho GTPase-activating protein 17"
}